{
  "term_id": "GO:0005231",
  "gene": "UniProtKB:Q9GZZ6",
  "gene_name": "Neuronal acetylcholine receptor subunit alpha-10",
  "term_label": "excitatory extracellular ligand-gated monoatomic ion channel activity",
  "gene_symbol": "CHRNA10"
}